positive regulation of meiotic cell cycle phase transition [GO:1901995] (biological process) Relationships: is a type of positive regulation of meiotic cell cycle [GO:0051446]; is a type of GO:1901989; is a type of GO:1901993; RO_0002213 meiotic cell cycle phase transition [GO:0044771] Also known as: activation of cell cycle transition, positive regulation of cell cycle transition, up regulation of cell cycle transition, up-regulation of cell cycle transition, upregulation of cell cycle transition, up regulation of meiotic cell cycle phase transition, up-regulation of meiotic cell cycle phase transition, upregulation of meiotic cell cycle phase transition, activation of meiotic cell cycle phase transition Subtypes: positive regulation of exit from meiosis [GO:0106062], positive regulation of G2/MI transition of meiotic cell cycle [GO:0110032], positive regulation of metaphase/anaphase transition of meiotic cell cycle [GO:1902104] References: PMID:22841721 Sources: GOC:TermGenie, GOC:mtg_cell_cycle Definition: Any process that activates or increases the frequency, rate or extent of meiotic cell cycle phase transition.